positive regulation of penicillin catabolic process [GO:0033249] (biological process) Also known as: positive regulation of penicillin breakdown, positive regulation of penicillin catabolism, positive regulation of penicillin degradation Sources: GOC:mah Relationships: is a type of positive regulation of catabolic process [GO:0009896]; is a type of positive regulation of penicillin metabolic process [GO:0033246]; is a type of GO:0033247; positively regulates penicillin catabolic process [GO:0042317] Definition: Any process that activates or increases the frequency, rate or extent of the chemical reactions and pathways leading to the breakdown of any antibiotic that contains the condensed beta-lactamthiazolidine ring system.